ABC-type thiamine transporter activity [GO:0048502] (molecular function) Also known as: thiamin pyrophosphate porter activity, thiamin pyrophosphate ABC transporter, thiamine ABC transporter, ATP-dependent thiamine transmembrane transporter activity, ATPase-coupled thiamine transmembrane transporter activity, TPP transporting ATPase activity, thiamin pyrophosphate transporting ATPase activity, thiamin-transporting ATPase activity, thiamine pyrophosphate-transporting ATPase activity, thiamine-transporting ATPase activity References: PMID:12175925, PMID:9535878 Sources: RHEA:29811 Relationships: is a type of thiamine transmembrane transporter activity [GO:0015234]; is_a ABC-type azole transporter activity [GO:0140394] Definition: Enables the transfer of a solute or solutes from one side of a membrane to the other according to the reaction: ATP + H2O + thiamine(out) = ADP + H+ + phosphate + thiamine(in).